{
  "gene_symbol": "GABRB1",
  "gene_name": "Gamma-aminobutyric acid receptor subunit beta-1",
  "gene": "UniProtKB:P18505",
  "term_label": "GABA-A receptor activity",
  "term_id": "GO:0004890"
}